oxidoreductase activity, acting on paired donors, with incorporation or reduction of molecular oxygen, reduced flavin or flavoprotein as one donor, and incorporation of one atom of oxygen [GO:0016712] (molecular function) Relationships: is a type of monooxygenase activity [GO:0004497]; is a type of oxidoreductase activity, acting on paired donors, with incorporation or reduction of molecular oxygen [GO:0016705] Definition: Catalysis of an oxidation-reduction (redox) reaction in which hydrogen or electrons are transferred from reduced flavin or flavoprotein and one other donor, and one atom of oxygen is incorporated into one donor. Subtypes: heme oxygenase (decyclizing) activity [GO:0004392], steroid 17-alpha-monooxygenase activity [GO:0004508], steroid 21-monooxygenase activity [GO:0004509], GO:0008123, testosterone 16-alpha-hydroxylase activity [GO:0008390], sterol 12-alpha-hydroxylase activity [GO:0008397], GO:0008726, nitrilotriacetate monooxygenase activity [GO:0018529], phenylacetate 2-hydroxylase activity [GO:0018631], dibenzothiophene monooxygenase activity [GO:0018640], (S)-limonene 3-monooxygenase activity [GO:0018674], (S)-limonene 6-monooxygenase activity [GO:0018675], (S)-limonene 7-monooxygenase activity [GO:0018676], dibenzothiophene sulfone monooxygenase (NADH) activity [GO:0018679], GO:0018684, GO:0033769, 2-hydroxyisoflavanone synthase activity [GO:0033770], flavanone 2-hydroxylase activity [GO:0033771], GO:0033773, GO:0033780, 24S-hydroxycholesterol 7-alpha-hydroxylase activity [GO:0033782], 25-hydroxycholesterol 7-alpha-hydroxylase activity [GO:0033783], ecdysteroid 25-hydroxylase activity [GO:0035302], indole-2-monooxygenase activity [GO:0036190], indolin-2-one monooxygenase activity [GO:0036191], GO:0036192, 2-hydroxy-1,4-benzoxazin-3-one monooxygenase activity [GO:0036193], taxoid 7beta-hydroxylase activity [GO:0036239], 3-hydroxy-9,10-secoandrosta-1,3,5(10)-triene-9,17-dione monooxygenase activity [GO:0036383], alkanal monooxygenase (FMN-linked) activity [GO:0047646], GO:0050051, linalool 8-monooxygenase activity [GO:0050056], 7-deoxyloganin 7-hydroxylase activity [GO:0050595], ent-kaurenoic acid monooxygenase activity [GO:0051777], (+)-menthofuran synthase activity [GO:0052582], ent-kaurene oxidase activity [GO:0052615], (R)-limonene 6-monooxygenase activity [GO:0052741], arachidonate omega-hydroxylase activity [GO:0052869], GO:0052871, 4-hydroxyphenylacetate 3-monooxygenase activity [GO:0052881], pipecolic acid N-hydroxylase [GO:0062047], GO:0070330, carotene epsilon hydroxylase activity [GO:0072374], thalianol hydroxylase activity [GO:0080014], GO:0090489, estrogen 16-alpha-hydroxylase activity [GO:0101020], estrogen 2-hydroxylase activity [GO:0101021], 22alpha-hydroxysteroid 23-monooxygenase activity [GO:0102097], GO:0102171, taxoid 2alpha-hydroxylase activity [GO:0102365], beta-amyrin 28-monooxygenase activity [GO:0102373], naringenin 2-hydroxylase activity [GO:0102469], GO:0102601, germacrene A acid 8beta-hydroxylase activity [GO:0102614], parthenolide synthase activity [GO:0102626], GO:0102627, GO:0102628, brassinolide synthase activity [GO:0102734], germacrene A hydroxylase activity [GO:0106223], labd-13Z-ene-9,15,16-triol synthase activity [GO:0106240], 3-chloro THPH synthase activity [GO:0106266], 3,5 dichloro-THPH synthase activity [GO:0106267], fatty acid omega-hydroxylase activity [GO:0120250], fatty acid omega-1 hydroxylase activity [GO:0120502], GO:0120511, farnesoate epoxidase activity [GO:0120512], homomethionine N-monooxygenase activity [GO:0120526], aflatoxin B synthase activity [GO:0140399], 7-deoxyloganate 7-hydroxylase activity [GO:0140989], steroid 22S-hydroxylase activity [GO:0160191] Sources: EC:1.14.14.- Also known as: aryl hydrocarbon hydroxylase activity, aryl-4-monooxygenase activity, cytochrome P450 CYP19, cytochrome p450 activity, flavoprotein monooxygenase activity, flavoprotein-linked monooxygenase activity, microsomal P-450, microsomal monooxygenase activity, microsomal p450 activity, unspecific monooxygenase activity, xenobiotic monooxygenase activity, substrate,reduced-flavoprotein:oxygen oxidoreductase (RH-hydroxylating or -epoxidizing)